{
  "term_id": "GO:0001164",
  "term_label": "RNA polymerase I core promoter sequence-specific DNA binding",
  "gene_symbol": "UBTFL6",
  "gene_name": "Putative upstream-binding factor 1-like protein 6",
  "gene": "UniProtKB:P0CB48"
}